{
  "term_id": "GO:0005544",
  "gene_name": "Cytosolic phospholipase A2 epsilon",
  "term_label": "calcium-dependent phospholipid binding",
  "gene": "UniProtKB:Q3MJ16",
  "gene_symbol": "PLA2G4E"
}